{
  "gene": "UniProtKB:Q6ZV50",
  "gene_name": "DNA-binding protein RFX8",
  "gene_symbol": "RFX8",
  "term_label": "nucleus",
  "term_id": "GO:0005634"
}